{
  "term_label": "mitochondrion",
  "term_id": "GO:0005739",
  "gene_name": "Nucleolar protein 3",
  "gene": "UniProtKB:O60936",
  "gene_symbol": "NOL3"
}